{
  "term_id": "GO:0017147",
  "term_label": "Wnt-protein binding",
  "gene": "UniProtKB:Q16827",
  "gene_name": "Receptor-type tyrosine-protein phosphatase O",
  "gene_symbol": "PTPRO"
}